{
  "term_label": "cytoplasm",
  "gene_symbol": "CAD",
  "gene": "UniProtKB:P27708",
  "gene_name": "CAD protein",
  "term_id": "GO:0005737"
}